{
  "gene_symbol": "IL1B",
  "term_label": "inflammatory response",
  "gene_name": "Interleukin-1 beta",
  "term_id": "GO:0006954",
  "gene": "UniProtKB:P01584"
}